{
  "term_label": "positive regulation of T cell mediated cytotoxicity",
  "gene": "UniProtKB:Q8TD07",
  "gene_symbol": "RAET1E",
  "term_id": "GO:0001916",
  "gene_name": "Retinoic acid early transcript 1E"
}